{
  "gene": "UniProtKB:P01762",
  "term_id": "UNKNOWN:0003",
  "gene_symbol": "IGHV3-11",
  "gene_name": "Immunoglobulin heavy variable 3-11",
  "term_label": "Unknown cellular component"
}